{
  "term_id": "GO:0099104",
  "gene": "UniProtKB:Q6ZSA7",
  "gene_symbol": "LRRC55",
  "term_label": "potassium channel activator activity",
  "gene_name": "Leucine-rich repeat-containing protein 55"
}